{
  "gene_symbol": "CLSPN",
  "term_id": "GO:0033314",
  "gene_name": "Claspin",
  "term_label": "mitotic DNA replication checkpoint signaling",
  "gene": "UniProtKB:Q9HAW4"
}